ds/ssDNA junction-specific dsDNA endonuclease activity [GO:0106332] (MF) Relationships: is a type of GO:1990238 Definition: Catalysis of the endonucleolytic cleavage of double-stranded DNA near a double-strand/single-strand DNA junction. References: PMID:14528010